{
  "gene_name": "Gem-associated protein 2",
  "term_id": "GO:0000387",
  "gene": "UniProtKB:O14893",
  "gene_symbol": "GEMIN2",
  "term_label": "spliceosomal snRNP assembly"
}